{
  "term_id": "GO:0098970",
  "gene": "UniProtKB:Q8WXS5",
  "term_label": "postsynaptic neurotransmitter receptor diffusion trapping",
  "gene_name": "Voltage-dependent calcium channel gamma-8 subunit",
  "gene_symbol": "CACNG8"
}